{
  "term_label": "Unknown molecular function",
  "gene_symbol": "Q8N2B8",
  "gene": "UniProtKB:Q8N2B8",
  "gene_name": "Putative uncharacterized protein FLJ33534",
  "term_id": "UNKNOWN:0001"
}